negative regulation of fractalkine production [GO:0032684] (biological process) Sources: GOC:mah Also known as: down regulation of fractalkine production, down-regulation of fractalkine production, downregulation of fractalkine production, negative regulation of CX3CL1 production, inhibition of fractalkine production, negative regulation of CX3CL1 biosynthesis, negative regulation of fractalkine biosynthetic process Relationships: is a type of GO:0032644; is a type of negative regulation of chemokine production [GO:0032682]; negatively regulates GO:0032603 Definition: Any process that stops, prevents, or reduces the frequency, rate, or extent of fractalkine production.